pyruvate, phosphate dikinase activity [GO:0050242] (molecular function) Also known as: ATP:pyruvate, phosphate phosphotransferase activity, PPDK, orthophosphate dikinase pyruvate, pyruvate, Pi dikinase activity, pyruvate,orthophosphate dikinase activity, pyruvate,phosphate dikinase activity, pyruvate-inorganic phosphate dikinase activity, pyruvate-phosphate dikinase (phosphorylating), pyruvate-phosphate dikinase activity, pyruvate-phosphate ligase activity, pyruvic-phosphate dikinase activity, pyruvic-phosphate ligase activity Relationships: is a type of phosphotransferase activity, paired acceptors [GO:0016781] Definition: Catalysis of the reaction: ATP + phosphate + pyruvate = AMP + diphosphate + 2 H+ + phosphoenolpyruvate. Sources: RHEA:10756